{
  "term_id": "GO:0003924",
  "gene_symbol": "BMS1",
  "gene": "UniProtKB:Q14692",
  "term_label": "GTPase activity",
  "gene_name": "Ribosome biogenesis protein BMS1 homolog"
}